inner dense plaque of desmosome [GO:0090637] (cellular component) Definition: The desmosomal part containing the C-termini of desmoplakins which interact with the keratin intermediate filaments, serving to tether the intermediate filaments to the plasma membrane. Relationships: is a type of GO:0110165; is part of desmosome [GO:0030057] References: PMID:20066089